foramen ovale closure [GO:0035922] (biological process) Definition: The morphogenetic process in which the foramen ovale closes after birth, to prevent blood flow between the right and left atria. In the fetal heart, the foramen ovale allows blood to enter the left atrium from the right atrium. Closure of the foramen ovale after birth stops this blood flow. References: PMID:19762328 Sources: GOC:BHF, GOC:vk, UBERON:0004754, Wikipedia:Foramen_ovale_(heart) Relationships: is a type of anatomical structure morphogenesis [GO:0009653]; is part of cardiac septum morphogenesis [GO:0060411] Also known as: foramen ovale of heart closure